{
  "gene": "UniProtKB:P31994",
  "term_label": "antibody-dependent cellular cytotoxicity",
  "term_id": "GO:0001788",
  "gene_name": "Low affinity immunoglobulin gamma Fc region receptor II-b",
  "gene_symbol": "FCGR2B"
}